{
  "term_label": "Unknown cellular component",
  "gene_name": "Cerebral cavernous malformations 2 protein-like",
  "term_id": "UNKNOWN:0003",
  "gene_symbol": "CCM2L",
  "gene": "UniProtKB:Q9NUG4"
}